{
  "term_label": "MHC class II protein complex",
  "gene_name": "HLA class II histocompatibility antigen, DQ alpha 2 chain",
  "gene": "UniProtKB:P01906",
  "gene_symbol": "HLA-DQA2",
  "term_id": "GO:0042613"
}